L-sorbose oxidase activity [GO:0050035] (molecular function) Relationships: is a type of GO:0016899 Also known as: L-sorbose:oxygen 5-oxidoreductase activity Sources: EC:1.1.3.11, RHEA:17853 Definition: Catalysis of the reaction: L-sorbose + O2 = 5-dehydro-D-fructose + H2O2.